{
  "gene_symbol": "WASH4P",
  "term_label": "WASH complex",
  "term_id": "GO:0071203",
  "gene": "UniProtKB:A8MWX3",
  "gene_name": "Putative WAS protein family homolog 4"
}